negative regulation of peptidyl-lysine acetylation [GO:2000757] (biological process) Relationships: is a type of negative regulation of protein acetylation [GO:1901984]; is a type of regulation of peptidyl-lysine acetylation [GO:2000756]; negatively regulates GO:0018394 Sources: GOC:obol Subtypes: negative regulation of N-terminal peptidyl-lysine acetylation [GO:2000760] Definition: Any process that stops, prevents or reduces the frequency, rate or extent of peptidyl-lysine acetylation.